{
  "term_id": "GO:0006508",
  "gene_symbol": "CPQ",
  "gene_name": "Carboxypeptidase Q",
  "gene": "UniProtKB:Q9Y646",
  "term_label": "proteolysis"
}